{
  "term_id": "UNKNOWN:0002",
  "term_label": "Unknown biological process",
  "gene_symbol": "C20orf85",
  "gene_name": "Uncharacterized protein C20orf85",
  "gene": "UniProtKB:Q9H1P6"
}